{
  "term_id": "GO:0006067",
  "term_label": "ethanol metabolic process",
  "gene_symbol": "ALDH2",
  "gene_name": "Aldehyde dehydrogenase, mitochondrial",
  "gene": "UniProtKB:P05091"
}